CCL2-activated CCR2 signaling pathway [GO:0038151] (biological process) Also known as: CCL2/CCR2 signaling pathway Sources: GOC:nhn, GOC:signaling Definition: The series of molecular signals initiated by the binding of the C-C chemokine CCL2 to a C-C chemokine type 2 receptor (CCR2) on the surface of a target cell, and ending with the regulation of a downstream cellular process, e.g. transcription. Relationships: is a type of chemokine (C-C motif) ligand 2 signaling pathway [GO:0038148]; is a type of GO:0038150